{
  "term_label": "group II metabotropic glutamate receptor activity",
  "gene": "UniProtKB:Q14832",
  "gene_name": "Metabotropic glutamate receptor 3",
  "term_id": "GO:0001641",
  "gene_symbol": "GRM3"
}